(Z,E)-alpha- farnesene synthase activity [GO:0102931] (molecular function) Relationships: is a type of GO:0016838 Definition: Catalysis of the reaction: 2-trans,6-trans-farnesyl diphosphate = (Z,E)-alpha-farnesene + diphosphoric acid. References: PMID:17140613 Sources: GOC:pz